{
  "term_label": "cytoplasmic translation",
  "term_id": "GO:0002181",
  "gene": "UniProtKB:Q9UET6",
  "gene_symbol": "FTSJ1",
  "gene_name": "Putative tRNA (cytidine(32)_guanosine(34)-2'-O)-methyltransferase"
}